{
  "gene": "UniProtKB:P08047",
  "term_id": "GO:0006357",
  "term_label": "regulation of transcription by RNA polymerase II",
  "gene_symbol": "SP1",
  "gene_name": "Transcription factor Sp1"
}